aspartate carbamoyltransferase activity [GO:0004070] (MF) Definition: Catalysis of the reaction: L-aspartate + carbamoyl phosphate = N-carbamoyl-L-aspartate + H+ + phosphate. Relationships: is a type of carboxyl- or carbamoyltransferase activity [GO:0016743] Sources: EC:2.1.3.2, RHEA:20013 Also known as: ATCase activity, L-aspartate transcarbamoylase activity, L-aspartate transcarbamylase activity, aspartate carbamyltransferase activity, aspartate transcarbamoylase activity, aspartate transcarbamylase activity, aspartic acid transcarbamoylase activity, aspartic carbamyltransferase activity, aspartic transcarbamylase activity, carbamoyl-phosphate:L-aspartate carbamoyltransferase activity, carbamoylaspartotranskinase activity, carbamylaspartotranskinase activity